{
  "gene_symbol": "CISD3",
  "term_id": "GO:0051604",
  "term_label": "protein maturation",
  "gene": "UniProtKB:P0C7P0",
  "gene_name": "CDGSH iron-sulfur domain-containing protein 3, mitochondrial"
}